inositol monophosphate 3-phosphatase activity [GO:0052832] (molecular function) Relationships: is a type of GO:0052834 Sources: RHEA:30739 Definition: Catalysis of the reaction: 1D-myo-inositol 3-phosphate + H2O = myo-inositol + phosphate.